symbiont-mediated suppression of host cytoplasmic pattern recognition receptor signaling pathway via inhibition of IKBKE activity [GO:0039724] (biological process) References: PMID:19153231, PMID:22532683, PMID:24173023 Definition: A process in which a symbiont interferes with, inhibits or disrupts a cytoplasmic pattern recognition receptor signaling pathway by reducing the activity of host I-kappa-B kinase epsilon (IKBKE/IKK-epsilon/IKK-E). Relationships: is a type of symbiont-mediated suppression of cytoplasmic pattern recognition receptor signaling pathway [GO:0039537] Also known as: suppression by virus of host viral-induced cytoplasmic pattern recognition receptor signaling pathway via inhibition of IKBKE activity, inhibition of host IKBKE by virus, suppression by virus of host IKBKE activity